{
  "term_label": "inositol-polyphosphate 5-phosphatase activity",
  "gene": "UniProtKB:O15357",
  "gene_symbol": "INPPL1",
  "gene_name": "Phosphatidylinositol 3,4,5-trisphosphate 5-phosphatase 2",
  "term_id": "GO:0004445"
}